mitochondrial disulfide relay system [GO:0160203] (BP) Relationships: is a type of GO:0006457; is part of GO:0045041 References: PMID:32936885, PMID:37159021 Also known as: MIA pathway, mitochondrial intermembrane space assembly pathway Definition: A protein folding process that facilitates the import of a subset of soluble proteins into mitochondrial intermembrane space via disulfide bond formation.